regulation of stomatal opening [GO:1902456] (biological process) Relationships: is a type of regulation of stomatal movement [GO:0010119]; regulates GO:1990069 Subtypes: negative regulation of stomatal opening [GO:1902457], positive regulation of stomatal opening [GO:1902458] Definition: Any process that modulates the frequency, rate or extent of stomatal opening. References: PMID:23766366 Sources: GOC:TermGenie